{
  "gene_name": "Putative disintegrin and metalloproteinase domain-containing protein 5",
  "gene_symbol": "ADAM5",
  "term_label": "Unknown biological process",
  "gene": "UniProtKB:Q6NVV9",
  "term_id": "UNKNOWN:0002"
}